{
  "gene": "UniProtKB:P51116",
  "gene_name": "RNA-binding protein FXR2",
  "gene_symbol": "FXR2",
  "term_id": "GO:0048170",
  "term_label": "positive regulation of long-term neuronal synaptic plasticity"
}